{
  "gene_symbol": "PCBD2",
  "gene_name": "Pterin-4-alpha-carbinolamine dehydratase 2",
  "term_label": "Unknown cellular component",
  "gene": "UniProtKB:Q9H0N5",
  "term_id": "UNKNOWN:0003"
}